lipase inhibitor activity [GO:0055102] (molecular function) Definition: Binds to and stops, prevents or reduces the activity of a lipase, an enzyme that catalyzes of the hydrolysis of a lipid. Sources: GOC:BHF, GOC:rl Relationships: is a type of enzyme inhibitor activity [GO:0004857]; negatively regulates lipase activity [GO:0016298] Subtypes: phospholipase inhibitor activity [GO:0004859]